ommochrome catabolic process [GO:0046153] (biological process) Definition: The chemical reactions and pathways resulting in the breakdown of ommochromes, any of a large group of natural polycyclic pigments commonly found in the Arthropoda, particularly in the ommatidia of the compound eye. Relationships: is_a catabolic process [GO:0009056]; is a type of eye pigment catabolic process [GO:0046151]; is a type of ommochrome metabolic process [GO:0046152]; is a type of ocellus pigment catabolic process [GO:0046159] Also known as: ommochrome breakdown, ommochrome catabolism, ommochrome degradation Sources: ISBN:0198506732